{
  "gene_name": "Phosphorylase b kinase gamma catalytic chain, liver_testis isoform",
  "gene": "UniProtKB:P15735",
  "term_id": "GO:0005964",
  "gene_symbol": "PHKG2",
  "term_label": "phosphorylase kinase complex"
}